negative regulation of amylopectin catabolic process [GO:2000946] (biological process) Also known as: negative regulation of Amylopectin catabolism Definition: Any process that stops, prevents or reduces the frequency, rate or extent of amylopectin catabolic process. Relationships: is a type of negative regulation of starch catabolic process [GO:2000882]; is a type of regulation of amylopectin catabolic process [GO:2000945]; negatively regulates amylopectin catabolic process [GO:2000897] Sources: GOC:mengo_curators